{
  "gene_name": "Sodium_hydrogen exchanger 2",
  "term_id": "GO:0098719",
  "gene": "UniProtKB:Q9UBY0",
  "term_label": "sodium ion import across plasma membrane",
  "gene_symbol": "SLC9A2"
}